sinoatrial node development [GO:0003163] (biological process) Also known as: SA node development, SAN development, sinus node development Relationships: is a type of atrial cardiac muscle tissue development [GO:0003228]; is part of cardiac conduction system development [GO:0003161] Sources: GOC:mtg_heart Definition: The process whose specific outcome is the progression of the sinoatrial (SA) node over time, from its formation to the mature structure. The SA node is part of the cardiac conduction system that controls the timing of heart muscle contraction. It relays electrical signals to the AV node.